{
  "gene_symbol": "CCDC80",
  "term_id": "GO:0005604",
  "gene_name": "Coiled-coil domain-containing protein 80",
  "gene": "UniProtKB:Q76M96",
  "term_label": "basement membrane"
}